positive regulation of hematopoietic progenitor cell differentiation [GO:1901534] (biological process) Also known as: activation of haematopoietic progenitor cell differentiation, activation of haemopoietic progenitor cell differentiation, positive regulation of haematopoietic progenitor cell differentiation, positive regulation of haemopoietic progenitor cell differentiation, positive regulation of hemopoietic progenitor cell differentiation, up regulation of haematopoietic progenitor cell differentiation, up regulation of haemopoietic progenitor cell differentiation, up regulation of hemopoietic progenitor cell differentiation, up-regulation of haematopoietic progenitor cell differentiation, up-regulation of haemopoietic progenitor cell differentiation, up-regulation of hemopoietic progenitor cell differentiation, upregulation of haematopoietic progenitor cell differentiation, upregulation of haemopoietic progenitor cell differentiation, upregulation of hemopoietic progenitor cell differentiation, activation of hemopoietic progenitor cell differentiation, activation of hematopoietic progenitor cell differentiation, up regulation of hematopoietic progenitor cell differentiation, up-regulation of hematopoietic progenitor cell differentiation, upregulation of hematopoietic progenitor cell differentiation Definition: Any process that activates or increases the frequency, rate or extent of hematopoietic progenitor cell differentiation. Sources: GOC:BHF, GOC:TermGenie, GOC:rl Relationships: is a type of positive regulation of cell differentiation [GO:0045597]; is a type of regulation of hematopoietic progenitor cell differentiation [GO:1901532]; RO_0002213 GO:0002244 Subtypes: positive regulation of hematopoietic stem cell differentiation [GO:1902038], positive regulation of myeloid progenitor cell differentiation [GO:1905455], positive regulation of lymphoid progenitor cell differentiation [GO:1905458]